{
  "term_id": "UNKNOWN:0001",
  "gene": "UniProtKB:O15127",
  "term_label": "Unknown molecular function",
  "gene_symbol": "SCAMP2",
  "gene_name": "Secretory carrier-associated membrane protein 2"
}